{
  "gene_symbol": "POPDC3",
  "term_label": "striated muscle cell differentiation",
  "term_id": "GO:0051146",
  "gene": "UniProtKB:Q9HBV1",
  "gene_name": "Popeye domain-containing protein 3"
}